{
  "gene": "UniProtKB:Q8IZ73",
  "term_id": "GO:0009982",
  "gene_symbol": "RPUSD2",
  "term_label": "pseudouridine synthase activity",
  "gene_name": "Pseudouridylate synthase RPUSD2"
}